nonassociative learning [GO:0046958] (biological process) Definition: A simple form of learning whereby the repeated presence of a stimulus leads to a change in the probability or strength of the response to that stimulus. There is no association of one type of stimulus with another, rather it is a generalized response to the environment. Sources: ISBN:0582227089 Relationships: is a type of learning [GO:0007612] Also known as: unconditional response Subtypes: GO:0046959, sensitization [GO:0046960], GO:0097270